regulation of small intestine smooth muscle contraction [GO:1904347] (biological process) Relationships: is a type of regulation of gastro-intestinal system smooth muscle contraction [GO:1904304]; RO_0002211 small intestine smooth muscle contraction [GO:1990770] Definition: Any process that modulates the frequency, rate or extent of small intestine smooth muscle contraction. References: PMID:11991626 Sources: GOC:TermGenie, GO_REF:0000058 Subtypes: negative regulation of small intestine smooth muscle contraction [GO:1904348], positive regulation of small intestine smooth muscle contraction [GO:1904349]